{
  "gene_name": "Cytohesin-2",
  "gene": "UniProtKB:Q99418",
  "term_label": "plasma membrane",
  "gene_symbol": "CYTH2",
  "term_id": "GO:0005886"
}